{
  "gene": "UniProtKB:A0A0J9YXY3",
  "term_id": "GO:0005886",
  "gene_symbol": "TRBV6-2",
  "gene_name": "T cell receptor beta variable 6-2",
  "term_label": "plasma membrane"
}